{
  "gene": "UniProtKB:Q8WWI1",
  "gene_symbol": "LMO7",
  "term_id": "UNKNOWN:0003",
  "term_label": "Unknown cellular component",
  "gene_name": "LIM domain only protein 7"
}